{
  "gene_symbol": "ACTR8",
  "term_label": "regulation of DNA-templated transcription",
  "term_id": "GO:0006355",
  "gene_name": "Actin-related protein 8",
  "gene": "UniProtKB:Q9H981"
}